{
  "term_id": "GO:0019809",
  "gene_symbol": "SAT1",
  "gene_name": "Diamine acetyltransferase 1",
  "gene": "UniProtKB:P21673",
  "term_label": "spermidine binding"
}